{
  "gene_symbol": "TLR10",
  "gene_name": "Toll-like receptor 10",
  "term_id": "GO:0071723",
  "term_label": "lipopeptide binding",
  "gene": "UniProtKB:Q9BXR5"
}